{
  "gene_symbol": "ARG1",
  "gene": "UniProtKB:P05089",
  "gene_name": "Arginase-1",
  "term_label": "cytosol",
  "term_id": "GO:0005829"
}